{
  "term_id": "UNKNOWN:0001",
  "term_label": "Unknown molecular function",
  "gene_name": "Ankyrin repeat domain-containing protein 31",
  "gene_symbol": "ANKRD31",
  "gene": "UniProtKB:Q8N7Z5"
}